{
  "gene": "UniProtKB:Q96NW4",
  "gene_symbol": "ANKRD27",
  "gene_name": "Ankyrin repeat domain-containing protein 27",
  "term_label": "early endosome",
  "term_id": "GO:0005769"
}